{
  "term_label": "metalloendopeptidase activity",
  "term_id": "GO:0004222",
  "gene_symbol": "TLL2",
  "gene_name": "Tolloid-like protein 2",
  "gene": "UniProtKB:Q9Y6L7"
}